{
  "gene": "UniProtKB:A4D263",
  "gene_name": "Spermatogenesis-associated protein 48",
  "term_label": "Unknown cellular component",
  "gene_symbol": "SPMIP7",
  "term_id": "UNKNOWN:0003"
}